{
  "gene_symbol": "SLC45A1",
  "term_id": "UNKNOWN:0002",
  "term_label": "Unknown biological process",
  "gene_name": "Proton-associated sugar transporter A",
  "gene": "UniProtKB:Q9Y2W3"
}